{
  "term_id": "GO:0005634",
  "gene_symbol": "RMND5A",
  "gene": "UniProtKB:Q9H871",
  "term_label": "nucleus",
  "gene_name": "E3 ubiquitin-protein transferase RMND5A"
}